{
  "gene": "UniProtKB:Q9H816",
  "gene_name": "5' exonuclease Apollo",
  "gene_symbol": "DCLRE1B",
  "term_id": "GO:0003684",
  "term_label": "damaged DNA binding"
}